{
  "gene_name": "Olfactory receptor 6Y1",
  "gene_symbol": "OR6Y1",
  "gene": "UniProtKB:Q8NGX8",
  "term_label": "detection of chemical stimulus involved in sensory perception of smell",
  "term_id": "GO:0050911"
}